{
  "gene_name": "E3 ubiquitin-protein ligase Midline-1",
  "gene": "UniProtKB:O15344",
  "term_label": "regulation of microtubule cytoskeleton organization",
  "gene_symbol": "MID1",
  "term_id": "GO:0070507"
}